quinolinate synthetase A activity [GO:0008987] (molecular function) Definition: Catalysis of the reaction: iminoaspartate + dihydroxy-acetone-phosphate = quinolinate + 2 H2O + phosphate. Sources: GOC:jl, MetaCyc:QUINOLINATE-SYNTHA-RXN Relationships: is a type of transferase activity, transferring alkyl or aryl (other than methyl) groups [GO:0016765]; is part of quinolinate biosynthetic process [GO:0019805]